RNA polymerase II complex recruiting activity [GO:0001139] (molecular function) Relationships: is a type of RNA polymerase II complex binding [GO:0000993]; is a type of GO:0030674; is part of RNA polymerase II preinitiation complex assembly [GO:0051123] Also known as: core RNA polymerase II recruiting transcription factor activity, transcription factor activity, core RNA polymerase II recruiting Definition: Binding to an RNA polymerase II (Pol II) complex, typically composed of twelve subunits, and with another protein, macromolecule, or complex, permitting those molecules to function in a coordinated way in order to facilitate the aggregation, arrangement and bonding together of proteins on an RNA polymerase II promoter DNA to form the transcriptional preinitiation complex (PIC), the formation of which is a prerequisite for transcription by RNA polymerase. References: PMID:16858867 Sources: GOC:txnOH